{
  "gene": "UniProtKB:Q9UHD4",
  "term_id": "GO:0006915",
  "term_label": "apoptotic process",
  "gene_symbol": "CIDEB",
  "gene_name": "Lipid transferase CIDEB"
}